{
  "term_id": "GO:0000978",
  "gene": "UniProtKB:P49335",
  "gene_name": "POU domain, class 3, transcription factor 4",
  "gene_symbol": "POU3F4",
  "term_label": "RNA polymerase II cis-regulatory region sequence-specific DNA binding"
}